positive regulation of polynucleotide adenylyltransferase activity [GO:1904247] (biological process) References: PMID:19460348 Sources: GOC:TermGenie, GOC:kmv, GO_REF:0000059 Definition: Any process that activates or increases the frequency, rate or extent of polynucleotide adenylyltransferase activity. Relationships: is a type of GO:0043085; is a type of regulation of transferase activity [GO:0051338]; positively regulates GO:1990817 Also known as: positive regulation of AMP polynucleotidylexotransferase activity, positive regulation of ATP-polynucleotide adenylyltransferase activity, positive regulation of ATP:polynucleotide adenylyltransferase activity, positive regulation of ATP:polynucleotidylexotransferase activity, positive regulation of NTP polymerase activity, positive regulation of RNA adenylating enzyme activity, positive regulation of adenosine triphosphate:ribonucleic acid adenylyltransferase activity, positive regulation of poly(A) hydrolase activity, positive regulation of poly(A) polymerase activity, positive regulation of poly(A) synthetase activity, positive regulation of poly-A polymerase activity, positive regulation of polyadenylate nucleotidyltransferase activity, positive regulation of polyadenylate polymerase activity, positive regulation of polyadenylate synthetase activity, positive regulation of polyadenylic acid polymerase activity, positive regulation of polyadenylic polymerase activity, positive regulation of terminal riboadenylate transferase activity, up regulation of AMP polynucleotidylexotransferase activity, up regulation of ATP-polynucleotide adenylyltransferase activity, up regulation of ATP:polynucleotide adenylyltransferase activity, up regulation of ATP:polynucleotidylexotransferase activity, up regulation of NTP polymerase activity, up regulation of RNA adenylating enzyme activity, up regulation of adenosine triphosphate:ribonucleic acid adenylyltransferase activity, up regulation of poly(A) hydrolase activity, up regulation of poly(A) polymerase activity, up regulation of poly(A) synthetase activity, up regulation of poly-A polymerase activity, up regulation of polyadenylate nucleotidyltransferase activity, up regulation of polyadenylate polymerase activity, up regulation of polyadenylate synthetase activity, up regulation of polyadenylic acid polymerase activity, up regulation of polyadenylic polymerase activity, up regulation of polynucleotide adenylyltransferase activity, up regulation of terminal riboadenylate transferase activity, up-regulation of AMP polynucleotidylexotransferase activity, up-regulation of ATP-polynucleotide adenylyltransferase activity, up-regulation of ATP:polynucleotide adenylyltransferase activity, up-regulation of ATP:polynucleotidylexotransferase activity, up-regulation of NTP polymerase activity, up-regulation of RNA adenylating enzyme activity, up-regulation of adenosine triphosphate:ribonucleic acid adenylyltransferase activity, up-regulation of poly(A) hydrolase activity, up-regulation of poly(A) polymerase activity, up-regulation of poly(A) synthetase activity, up-regulation of poly-A polymerase activity, up-regulation of polyadenylate nucleotidyltransferase activity, up-regulation of polyadenylate polymerase activity, up-regulation of polyadenylate synthetase activity, up-regulation of polyadenylic acid polymerase activity, up-regulation of polyadenylic polymerase activity, up-regulation of polynucleotide adenylyltransferase activity, up-regulation of terminal riboadenylate transferase activity, upregulation of AMP polynucleotidylexotransferase activity, upregulation of ATP-polynucleotide adenylyltransferase activity, upregulation of ATP:polynucleotide adenylyltransferase activity, upregulation of ATP:polynucleotidylexotransferase activity, upregulation of NTP polymerase activity, upregulation of RNA adenylating enzyme activity, upregulation of adenosine triphosphate:ribonucleic acid adenylyltransferase activity, upregulation of poly(A) hydrolase activity, upregulation of poly(A) polymerase activity, upregulation of poly(A) synthetase activity, upregulation of poly-A polymerase activity, upregulation of polyadenylate nucleotidyltransferase activity, upregulation of polyadenylate polymerase activity, upregulation of polyadenylate synthetase activity, upregulation of polyadenylic acid polymerase activity, upregulation of polyadenylic polymerase activity, upregulation of polynucleotide adenylyltransferase activity, upregulation of terminal riboadenylate transferase activity, activation of AMP polynucleotidylexotransferase activity, activation of ATP-polynucleotide adenylyltransferase activity, activation of ATP:polynucleotide adenylyltransferase activity, activation of ATP:polynucleotidylexotransferase activity, activation of NTP polymerase activity, activation of RNA adenylating enzyme activity, activation of adenosine triphosphate:ribonucleic acid adenylyltransferase activity, activation of poly(A) hydrolase activity, activation of poly(A) polymerase activity, activation of poly(A) synthetase activity, activation of poly-A polymerase activity, activation of polyadenylate nucleotidyltransferase activity, activation of polyadenylate polymerase activity, activation of polyadenylate synthetase activity, activation of polyadenylic acid polymerase activity, activation of polyadenylic polymerase activity, activation of polynucleotide adenylyltransferase activity, activation of terminal riboadenylate transferase activity, activation of RNA formation factors, PF1, positive regulation of RNA formation factors, PF1, up regulation of RNA formation factors, PF1, up-regulation of RNA formation factors, PF1, upregulation of RNA formation factors, PF1